{
  "gene_name": "Krueppel-like factor 15",
  "gene_symbol": "KLF15",
  "term_label": "DNA-binding transcription factor activity, RNA polymerase II-specific",
  "gene": "UniProtKB:Q9UIH9",
  "term_id": "GO:0000981"
}